{
  "term_id": "UNKNOWN:0002",
  "term_label": "Unknown biological process",
  "gene": "UniProtKB:Q5JWR5",
  "gene_symbol": "DOP1A",
  "gene_name": "Protein dopey-1"
}